{
  "gene": "UniProtKB:P47890",
  "gene_name": "Olfactory receptor 1G1",
  "term_label": "signal transduction",
  "gene_symbol": "OR1G1",
  "term_id": "GO:0007165"
}